{
  "term_label": "sodium channel regulator activity",
  "gene_name": "FXYD domain-containing ion transport regulator 6",
  "gene_symbol": "FXYD6",
  "gene": "UniProtKB:Q9H0Q3",
  "term_id": "GO:0017080"
}